{
  "gene_symbol": "SH3TC1",
  "gene": "UniProtKB:Q8TE82",
  "gene_name": "SH3 domain and tetratricopeptide repeat-containing protein 1",
  "term_id": "UNKNOWN:0002",
  "term_label": "Unknown biological process"
}